6-methylthiopropyl glucosinolate S-oxygenase activity [GO:0080105] (molecular function) Definition: Catalysis of the reaction: 6-methylthiopropyl-glucosinolate = 6-methylsulfinylpropyl-glucosinolate. References: PMID:18799661 Relationships: is a type of oxidoreductase activity, acting on paired donors, with incorporation or reduction of molecular oxygen [GO:0016705]